{
  "gene_name": "Thyroid receptor-interacting protein 11",
  "gene": "UniProtKB:Q15643",
  "term_id": "GO:0006888",
  "gene_symbol": "TRIP11",
  "term_label": "endoplasmic reticulum to Golgi vesicle-mediated transport"
}